{
  "gene": "UniProtKB:P49917",
  "term_id": "GO:0005958",
  "term_label": "DNA-dependent protein kinase-DNA ligase 4 complex",
  "gene_name": "DNA ligase 4",
  "gene_symbol": "LIG4"
}